{
  "gene_name": "Zinc finger protein 391",
  "term_label": "RNA polymerase II transcription regulatory region sequence-specific DNA binding",
  "gene_symbol": "ZNF391",
  "gene": "UniProtKB:Q9UJN7",
  "term_id": "GO:0000977"
}